{
  "gene": "UniProtKB:Q9BYS1",
  "term_id": "UNKNOWN:0003",
  "gene_name": "Keratin-associated protein 1-5",
  "term_label": "Unknown cellular component",
  "gene_symbol": "KRTAP1-5"
}